{
  "gene_name": "Distal membrane-arm assembly complex protein 1",
  "gene": "UniProtKB:Q96GE9",
  "gene_symbol": "DMAC1",
  "term_id": "GO:0005743",
  "term_label": "mitochondrial inner membrane"
}